{
  "gene": "UniProtKB:Q8N6W0",
  "term_id": "GO:0000381",
  "gene_symbol": "CELF5",
  "term_label": "regulation of alternative mRNA splicing, via spliceosome",
  "gene_name": "CUGBP Elav-like family member 5"
}